{
  "gene_symbol": "THRSP",
  "term_label": "molecular function inhibitor activity",
  "gene_name": "Thyroid hormone-inducible hepatic protein",
  "gene": "UniProtKB:Q92748",
  "term_id": "GO:0140678"
}